(3R)-citramalyl-CoA lyase activity [GO:0044101] (molecular function) Definition: Catalysis of the reaction: (3R)-citramalyl-CoA = pyruvate + acetyl-CoA. Sources: GOC:jl Also known as: R-citramalyl-CoA lyase activity, Ccl Relationships: is_a oxo-acid-lyase activity [GO:0016833]